tolerance induction to self antigen [GO:0002513] (biological process) Sources: GOC:jal, GO_REF:0000022, ISBN:0781735149 Subtypes: GO:0002466, central tolerance induction to self antigen [GO:0002509] Regulation: regulated by regulation of tolerance induction to self antigen [GO:0002649]; RO_0002212 by negative regulation of tolerance induction to self antigen [GO:0002650]; positively regulated by GO:0002651 Definition: Tolerance induction directed at self antigens. Relationships: is a type of tolerance induction [GO:0002507]